CD8-positive, alpha-beta cytotoxic T cell extravasation [GO:0035698] (biological process) Regulation: regulated by regulation of CD8-positive, alpha-beta cytotoxic T cell extravasation [GO:2000452]; negatively regulated by GO:2000453; positively regulated by positive regulation of CD8-positive, alpha-beta cytotoxic T cell extravasation [GO:2000454] Sources: CL:0000794, GOC:BHF Relationships: is a type of GO:0035697 Definition: The migration of a CD8-positive, alpha-beta cytotoxic T cell from the blood vessels into the surrounding tissue.